{
  "term_id": "GO:0070857",
  "term_label": "regulation of bile acid biosynthetic process",
  "gene_name": "Fibroblast growth factor receptor 4",
  "gene": "UniProtKB:P22455",
  "gene_symbol": "FGFR4"
}